transforming growth factor beta ligand-receptor complex [GO:0070021] (cellular component) Relationships: is a type of plasma membrane signaling receptor complex [GO:0098802]; is a type of GO:1902554 Sources: GOC:curators Definition: A protein complex that is formed by the association of a TGF-beta dimeric ligand with 2 molecules of each receptor molecule, TGF-beta type I receptor and TGF-beta type II receptor. The receptor molecules may form homo- or heterodimers but only once bound by the ligand. Also known as: TGF-beta ligand-receptor complex, TGFb ligand-receptor complex, TGFbeta ligand-receptor complex, TGF-beta 1:type II receptor:type I receptor complex, TGF-beta receptor II-TGF-beta receptor I-TGF-beta1 complex, TGF-beta1 ligand-receptor complex, TGF-beta1-beta2 ligand-receptor complex, TGF-beta1-type II receptor-type I receptor complex, TGF-beta2 ligand-receptor complex, TGFbeta1 ligand-receptor complex, TGFbeta1-beta2 ligand-receptor complex, TGFbeta2 ligand-receptor complex, transforming growth factor beta1-type II receptor-type I receptor complex